{
  "term_label": "coreceptor activity",
  "gene_name": "Hemojuvelin",
  "gene": "UniProtKB:Q6ZVN8",
  "term_id": "GO:0015026",
  "gene_symbol": "HJV"
}